{
  "gene_name": "S-adenosylmethionine-dependent nucleotide dehydratase RSAD2",
  "gene": "UniProtKB:Q8WXG1",
  "gene_symbol": "RSAD2",
  "term_label": "mitochondrion",
  "term_id": "GO:0005739"
}